{
  "gene_name": "Sulfotransferase 6B1",
  "term_id": "GO:0005737",
  "gene": "UniProtKB:Q6IMI4",
  "gene_symbol": "SULT6B1",
  "term_label": "cytoplasm"
}